{
  "term_id": "GO:0007411",
  "gene_name": "Kinesin heavy chain isoform 5A",
  "term_label": "axon guidance",
  "gene": "UniProtKB:Q12840",
  "gene_symbol": "KIF5A"
}